{
  "gene_name": "Semaphorin-5B",
  "gene_symbol": "SEMA5B",
  "gene": "UniProtKB:Q9P283",
  "term_label": "plasma membrane",
  "term_id": "GO:0005886"
}